{
  "term_id": "GO:0005634",
  "gene_name": "Zinc finger protein 292",
  "gene_symbol": "ZNF292",
  "term_label": "nucleus",
  "gene": "UniProtKB:O60281"
}